{
  "gene": "UniProtKB:Q14159",
  "gene_symbol": "SPIDR",
  "term_id": "UNKNOWN:0001",
  "term_label": "Unknown molecular function",
  "gene_name": "DNA repair-scaffolding protein"
}